{
  "term_label": "phospholipase A2 activity",
  "term_id": "GO:0004623",
  "gene_name": "Phospholipase ABHD3",
  "gene_symbol": "ABHD3",
  "gene": "UniProtKB:Q8WU67"
}